negative regulation of T cell tolerance induction to tumor cell [GO:0002847] (biological process) Also known as: down regulation of T cell tolerance induction to tumor cell, down-regulation of T cell tolerance induction to tumor cell, downregulation of T cell tolerance induction to tumor cell, inhibition of T cell tolerance induction to tumor cell Relationships: is a type of GO:0002841; is a type of GO:0002844; is a type of regulation of T cell tolerance induction to tumor cell [GO:0002846]; is a type of GO:0002850; negatively regulates T cell tolerance induction to tumor cell [GO:0002411] Definition: Any process that stops, prevents, or reduces the frequency, rate, or extent of T cell tolerance induction to tumor cell. Sources: GOC:add